pentachlorophenol monooxygenase activity [GO:0018677] (molecular function) Relationships: is a type of oxidoreductase activity, acting on paired donors, with incorporation or reduction of molecular oxygen, NAD(P)H as one donor, and incorporation of one atom of oxygen [GO:0016709] Definition: Catalysis of the reaction: pentachlorophenol + NADPH + H+ + O2 = tetrachlorohydroquinone + NADP+ + chloride. Also known as: pentachlorophenol 4-monooxygenase activity, pentachlorophenol hydroxylase activity, PCB 4-monooxygenase activity, PCB4MO activity, PCP hydroxylase activity, PcpB, pentachlorophenol dechlorinase activity, pentachlorophenol dehalogenase activity, pentachlorophenol,NADPH:oxygen oxidoreductase (hydroxylating, dechlorinating) Sources: EC:1.14.13.50